{
  "gene": "UniProtKB:Q15940",
  "term_label": "DNA-binding transcription factor activity, RNA polymerase II-specific",
  "gene_name": "Putative zinc finger protein 726P1",
  "term_id": "GO:0000981",
  "gene_symbol": "ZNF726P1"
}